{
  "gene_symbol": "CBLN4",
  "term_label": "extracellular space",
  "gene": "UniProtKB:Q9NTU7",
  "term_id": "GO:0005615",
  "gene_name": "Cerebellin-4"
}